{
  "term_id": "UNKNOWN:0003",
  "gene": "UniProtKB:A0A075B6W5",
  "term_label": "Unknown cellular component",
  "gene_name": "T cell receptor alpha variable 23_delta variable 6",
  "gene_symbol": "TRAV23DV6"
}